cytoskeleton-dependent cytokinesis [GO:0061640] (biological process) Definition: A cytokinesis that involves the function of a set of proteins that are part of the microfilament or microtubule cytoskeleton. Sources: GOC:dph Relationships: is a type of cytokinesis [GO:0000910] Subtypes: mitotic cytokinesis [GO:0000281], meiotic cytokinesis [GO:0033206]